{
  "gene_symbol": "SPATA31F1",
  "gene": "UniProtKB:Q6ZU69",
  "gene_name": "Protein SPATA31F1",
  "term_id": "UNKNOWN:0001",
  "term_label": "Unknown molecular function"
}